lactam catabolic process [GO:0072340] (biological process) Definition: The chemical reactions and pathways resulting in the breakdown of lactams, any cyclic amides of amino carboxylic acids, having a 1-azacycloalkan-2-one structure, or analogues having unsaturation or heteroatoms replacing one or more carbon atoms of the ring. Relationships: is_a GO:0009056; is a type of GO:0072338 Also known as: cellular lactam breakdown, cellular lactam catabolic process, cellular lactam catabolism, cellular lactam degradation Sources: GOC:mah Subtypes: creatinine catabolic process [GO:0006602], caprolactam catabolic process [GO:0019384], GO:0030655, emericellamide catabolic process [GO:1900556], pseurotin A catabolic process [GO:1900789]